{
  "gene_symbol": "TBX15",
  "term_label": "regulation of transcription by RNA polymerase II",
  "term_id": "GO:0006357",
  "gene_name": "T-box transcription factor TBX15",
  "gene": "UniProtKB:Q96SF7"
}